{
  "term_id": "GO:0000981",
  "gene_name": "Transcription factor Jun",
  "gene_symbol": "JUN",
  "gene": "UniProtKB:P05412",
  "term_label": "DNA-binding transcription factor activity, RNA polymerase II-specific"
}